{
  "gene": "UniProtKB:P05106",
  "term_id": "GO:0009986",
  "term_label": "cell surface",
  "gene_symbol": "ITGB3",
  "gene_name": "Integrin beta-3"
}